benzene catabolic process [GO:1900996] (biological process) Relationships: is a type of GO:0018910; is a type of GO:0120253 Also known as: benzene breakdown, benzene catabolism, benzene degradation Sources: GOC:TermGenie, GOC:yaf, UniPathway:UPA00272 Definition: The chemical reactions and pathways resulting in the breakdown of benzene.